{
  "gene": "UniProtKB:Q3LI77",
  "gene_symbol": "KRTAP13-4",
  "term_label": "Unknown molecular function",
  "term_id": "UNKNOWN:0001",
  "gene_name": "Keratin-associated protein 13-4"
}